fumarate metabolic process [GO:0006106] (biological process) Relationships: is a type of dicarboxylic acid metabolic process [GO:0043648] Definition: The chemical reactions and pathways involving fumarate, the anion of trans-1,2-ethenedicarboxylic acid, the diastereoisomer of maleate. It is a key intermediate in metabolism and is formed in the TCA cycle from succinate and converted into malate. Sources: ISBN:0198506732 Subtypes: GO:0019445 Also known as: fumarate metabolism